regulation of acetylcholine secretion, neurotransmission [GO:0014056] (biological process) Definition: Any process that modulates the frequency, rate or extent of the regulated release of acetylcholine. Relationships: is a type of regulation of synaptic transmission, cholinergic [GO:0032222]; is a type of regulation of neurotransmitter secretion [GO:0046928]; is_a regulation of amine transport [GO:0051952]; regulates GO:0014055 Subtypes: GO:0014057, negative regulation of acetylcholine secretion, neurotransmission [GO:0014058] Sources: GOC:ef